{
  "gene": "UniProtKB:Q7RTX0",
  "term_label": "plasma membrane",
  "gene_symbol": "TAS1R3",
  "gene_name": "Taste receptor type 1 member 3",
  "term_id": "GO:0005886"
}